2,5-diketocamphane 1,2-monooxygenase [GO:0018684] (molecular function) Definition: Catalysis of the reaction: 1R,4R)-bornane-2,5-dione + FMNH2 + O2 = (1R,4R)-5-oxo-1,2-campholide + FMN + H+ + H2O. Also known as: camphor 1,2-monooxygenase activity, (+)-camphor,reduced-rubredoxin:oxygen oxidoreductase (1,2-lactonizing), 2,5-diketocamphane lactonizing enzyme activity, camphor ketolactonase I activity References: PMID:3944058, PMID:8515237 Sources: RHEA:34415 Relationships: is a type of oxidoreductase activity, acting on paired donors, with incorporation or reduction of molecular oxygen, reduced flavin or flavoprotein as one donor, and incorporation of one atom of oxygen [GO:0016712]